{
  "gene": "UniProtKB:Q8N7S6",
  "gene_symbol": "ARIH2OS",
  "term_label": "Unknown molecular function",
  "gene_name": "Uncharacterized protein ARIH2OS",
  "term_id": "UNKNOWN:0001"
}